{
  "gene_symbol": "RRN3P1",
  "gene_name": "Putative RRN3-like protein RRN3P1",
  "term_id": "UNKNOWN:0001",
  "gene": "UniProtKB:Q2M238",
  "term_label": "Unknown molecular function"
}